dimeric ribonuclease P complex [GO:0030680] (cellular component) Relationships: is a type of ribonuclease P complex [GO:0030677] Also known as: dimeric RNase P complex Definition: A ribonuclease P complex that contains a single RNA molecule that is necessary and usually sufficient for catalysis, and a single protein molecule. Examples of this complex are found in Bacterial species. References: PMID:12045094 Sources: GOC:mah